establishment of protein localization to endoplasmic reticulum [GO:0072599] (biological process) Definition: The directed movement of a protein to a specific location in the endoplasmic reticulum. Subtypes: protein targeting to ER [GO:0045047], establishment of protein localization to endoplasmic reticulum membrane [GO:0097051] Sources: GOC:mah Also known as: establishment of protein localisation to ER, establishment of protein localisation to endoplasmic reticulum, establishment of protein localization in endoplasmic reticulum, establishment of protein localization to ER Relationships: is a type of GO:0072594